{
  "term_label": "guanyl-nucleotide exchange factor activity",
  "gene_symbol": "LAMTOR1",
  "term_id": "GO:0005085",
  "gene": "UniProtKB:Q6IAA8",
  "gene_name": "Ragulator complex protein LAMTOR1"
}